DNA replication preinitiation complex [GO:0031261] (CC) References: PMID:12694535, PMID:15194812, PMID:17230184 Sources: GOC:bf, GOC:hjd, GOC:jl, GOC:pr, GOC:rb Relationships: is a type of GO:0032993; is a type of nuclear protein-containing complex [GO:0140513]; is part of nucleoplasm [GO:0005654]; has part GO:0005656 Definition: A protein-DNA complex assembled at eukaryotic DNA replication origins immediately prior to the initiation of DNA replication. The preinitiation complex is formed by the assembly of additional proteins onto an existing prereplicative complex. In budding yeast, the additional proteins might include Cdc45p, Sld2p, Sld3p, Dpb11p, DNA polymerases, and others; in fission yeast the GINS complex is present. Also known as: pre-IC Subtypes: GO:0000811, CMG complex [GO:0071162]